{
  "term_id": "GO:0005929",
  "gene": "UniProtKB:Q9HBA0",
  "gene_symbol": "TRPV4",
  "gene_name": "Transient receptor potential cation channel subfamily V member 4",
  "term_label": "cilium"
}